response to reactive oxygen species [GO:0000302] (biological process) Also known as: response to AOS, response to ROI, response to ROS, response to active oxygen species, response to reactive oxidative species, response to reactive oxygen intermediate Sources: GOC:krc Regulation: regulated by GO:1901031; negatively regulated by negative regulation of response to reactive oxygen species [GO:1901032]; positively regulated by positive regulation of response to reactive oxygen species [GO:1901033] Subtypes: response to singlet oxygen [GO:0000304], GO:0000305, GO:0010193, cellular response to reactive oxygen species [GO:0034614], response to hydrogen peroxide [GO:0042542], response to hypochlorite [GO:1901530] Definition: Any process that results in a change in state or activity of a cell or an organism (in terms of movement, secretion, enzyme production, gene expression, etc.) as a result of a reactive oxygen species stimulus. Reactive oxygen species include singlet oxygen, superoxide, and oxygen free radicals. Relationships: is a type of GO:0006979; is a type of response to oxygen-containing compound [GO:1901700]